{
  "term_id": "GO:0005615",
  "term_label": "extracellular space",
  "gene_symbol": "ECM1",
  "gene": "UniProtKB:Q16610",
  "gene_name": "Extracellular matrix protein 1"
}